{
  "term_id": "GO:0005789",
  "gene_name": "ERO1-like protein alpha",
  "term_label": "endoplasmic reticulum membrane",
  "gene_symbol": "ERO1A",
  "gene": "UniProtKB:Q96HE7"
}